{
  "gene_symbol": "MTARC1",
  "gene": "UniProtKB:Q5VT66",
  "term_id": "GO:0008940",
  "gene_name": "Mitochondrial amidoxime-reducing component 1",
  "term_label": "nitrate reductase activity"
}